{
  "gene": "UniProtKB:Q15466",
  "term_label": "cytoplasm",
  "gene_name": "Nuclear receptor subfamily 0 group B member 2",
  "term_id": "GO:0005737",
  "gene_symbol": "NR0B2"
}